{
  "gene": "UniProtKB:O95772",
  "gene_symbol": "STARD3NL",
  "term_label": "endoplasmic reticulum membrane",
  "gene_name": "STARD3 N-terminal-like protein",
  "term_id": "GO:0005789"
}